{
  "term_id": "GO:0000978",
  "gene": "UniProtKB:O14948",
  "gene_symbol": "TFEC",
  "gene_name": "Transcription factor EC",
  "term_label": "RNA polymerase II cis-regulatory region sequence-specific DNA binding"
}